{
  "gene_name": "Putative uncharacterized protein COL25A1-DT",
  "gene_symbol": "COL25A1-DT",
  "term_id": "UNKNOWN:0002",
  "term_label": "Unknown biological process",
  "gene": "UniProtKB:Q6ZST2"
}